regulation of mRNA stability involved in response to oxidative stress [GO:2000815] (biological process) Definition: A process of regulation of mRNA stability that is involved in a response to oxidative stress. Sources: GOC:obol Relationships: is a type of GO:0010610; is part of response to oxidative stress [GO:0006979]